pyruvate carboxylase activity [GO:0004736] (molecular function) Sources: EC:6.4.1.1, RHEA:20844 Definition: Catalysis of the reaction: ATP + bicarbonate + pyruvate = ADP + 2 H+ + oxaloacetate + phosphate. Relationships: is a type of GO:0016885 Also known as: pyruvate:carbon-dioxide ligase (ADP-forming), pyruvic carboxylase activity